{
  "gene": "UniProtKB:Q9BRH9",
  "term_label": "RNA polymerase II cis-regulatory region sequence-specific DNA binding",
  "gene_symbol": "ZNF251",
  "gene_name": "Zinc finger protein 251",
  "term_id": "GO:0000978"
}